{
  "gene": "UniProtKB:Q9NZP5",
  "gene_name": "Olfactory receptor 5AC2",
  "term_label": "Unknown biological process",
  "term_id": "UNKNOWN:0002",
  "gene_symbol": "OR5AC2"
}